{
  "gene_name": "Guanine nucleotide-binding protein G(I)_G(S)_G(O) subunit gamma-5",
  "term_label": "heterotrimeric G-protein complex",
  "term_id": "GO:0005834",
  "gene": "UniProtKB:P63218",
  "gene_symbol": "GNG5"
}